geranyl diphosphate biosynthetic process [GO:0033384] (biological process) Also known as: geranyl diphosphate anabolism, geranyl diphosphate biosynthesis, geranyl diphosphate formation, geranyl diphosphate synthesis, geranyldiphosphate biosynthetic process Relationships: is a type of phospholipid biosynthetic process [GO:0008654]; is_a terpenoid biosynthetic process [GO:0016114]; is a type of geranyl diphosphate metabolic process [GO:0033383] Sources: GOC:mah, MetaCyc:PWY-5122 Definition: The chemical reactions and pathways resulting in the formation of geranyl diphosphate.